{
  "gene": "UniProtKB:Q9UBK8",
  "term_label": "methionine biosynthetic process",
  "gene_symbol": "MTRR",
  "term_id": "GO:0009086",
  "gene_name": "Methionine synthase reductase"
}